{
  "term_label": "Unknown biological process",
  "gene_name": "RNA-binding protein 39",
  "gene_symbol": "RBM39",
  "gene": "UniProtKB:Q14498",
  "term_id": "UNKNOWN:0002"
}